{
  "term_label": "calcium ion binding",
  "gene_symbol": "PLA2G4C",
  "gene_name": "Cytosolic phospholipase A2 gamma",
  "gene": "UniProtKB:Q9UP65",
  "term_id": "GO:0005509"
}